{
  "term_label": "sulfide:quinone oxidoreductase activity",
  "gene": "UniProtKB:Q9Y6N5",
  "term_id": "GO:0070224",
  "gene_symbol": "SQOR",
  "gene_name": "Sulfide:quinone oxidoreductase, mitochondrial"
}